{
  "gene": "UniProtKB:P22760",
  "term_id": "GO:0010898",
  "gene_name": "Arylacetamide deacetylase",
  "term_label": "positive regulation of triglyceride catabolic process",
  "gene_symbol": "AADAC"
}